{
  "gene_name": "Interferon lambda-2",
  "gene": "UniProtKB:Q8IZJ0",
  "gene_symbol": "IFNL2",
  "term_id": "GO:0045087",
  "term_label": "innate immune response"
}